positive regulation of bioluminescence [GO:1905087] (biological process) Relationships: is a type of positive regulation of metabolic process [GO:0009893]; is a type of GO:1905085; positively regulates bioluminescence [GO:0008218] Also known as: up regulation of bioluminescence, up-regulation of bioluminescence, upregulation of bioluminescence, activation of bioluminescence Definition: Any process that activates or increases the frequency, rate or extent of bioluminescence. References: PMID:10913092 Sources: GOC:BHF, GOC:TermGenie, GOC:rph, GO_REF:0000058